lung pattern specification process [GO:0060432] (biological process) Sources: GOC:dph Relationships: is_a pattern specification process [GO:0007389]; is part of lung development [GO:0030324] Definition: Any developmental process that results in the creation of defined areas or spaces within the lung, to which cells respond and eventually are instructed to differentiate. Subtypes: lung proximal/distal axis specification [GO:0061115]